regulation of ascus development [GO:0075318] (BP) Relationships: is a type of GO:0075260; regulates ascus development [GO:0075317] Sources: GOC:pamgo_curators Subtypes: positive regulation of ascus development [GO:0075319], negative regulation of ascus development [GO:0075320] Definition: Any process that modulates the frequency, rate or extent of ascus development, a process that leads to the formation of basidium, a sac-like structure produced by fungi of the phylum Ascomycota (sac fungi) in which sexually produced spores (ascospores), usually four or eight in number, are formed.